{
  "gene": "UniProtKB:O94805",
  "term_id": "GO:0016514",
  "term_label": "SWI/SNF complex",
  "gene_symbol": "ACTL6B",
  "gene_name": "Actin-like protein 6B"
}